{
  "gene_symbol": "POTEI",
  "gene_name": "POTE ankyrin domain family member I",
  "term_label": "actin cytoskeleton",
  "term_id": "GO:0015629",
  "gene": "UniProtKB:P0CG38"
}